{
  "gene_symbol": "SNX15",
  "term_label": "Unknown biological process",
  "gene": "UniProtKB:Q9NRS6",
  "term_id": "UNKNOWN:0002",
  "gene_name": "Sorting nexin-15"
}